{
  "term_id": "UNKNOWN:0002",
  "gene": "UniProtKB:Q5R3K3",
  "gene_name": "Calcium homeostasis modulator protein 6",
  "gene_symbol": "CALHM6",
  "term_label": "Unknown biological process"
}